positive regulation of presynaptic membrane organization [GO:1901631] (biological process) References: PMID:22426000 Sources: GOC:TermGenie Relationships: is a type of GO:0051130; is a type of GO:1901629; positively regulates GO:0097090 Also known as: positive regulation of pre-synaptic membrane organization, positive regulation of presynaptic membrane organisation, up regulation of presynaptic membrane organisation, up regulation of presynaptic membrane organization, up-regulation of presynaptic membrane organisation, up-regulation of presynaptic membrane organization, upregulation of presynaptic membrane organisation, upregulation of presynaptic membrane organization, activation of presynaptic membrane organisation, activation of presynaptic membrane organization Definition: Any process that activates or increases the frequency, rate or extent of presynaptic membrane organization.